{
  "term_id": "GO:0016684",
  "gene": "UniProtKB:P58004",
  "gene_symbol": "SESN2",
  "gene_name": "Sestrin-2",
  "term_label": "oxidoreductase activity, acting on peroxide as acceptor"
}